{
  "gene_symbol": "ATM",
  "term_label": "protein serine/threonine kinase activity",
  "gene_name": "Serine-protein kinase ATM",
  "term_id": "GO:0004674",
  "gene": "UniProtKB:Q13315"
}